{
  "term_label": "Unknown cellular component",
  "gene_name": "Transmembrane protein 200B",
  "gene": "UniProtKB:Q69YZ2",
  "term_id": "UNKNOWN:0003",
  "gene_symbol": "TMEM200B"
}